{
  "gene_symbol": "DLK2",
  "term_label": "Unknown cellular component",
  "gene": "UniProtKB:Q6UY11",
  "term_id": "UNKNOWN:0003",
  "gene_name": "Protein delta homolog 2"
}